canonical Wnt signaling pathway [GO:0060070] (biological process) Regulation: regulated by regulation of canonical Wnt signaling pathway [GO:0060828]; negatively regulated by negative regulation of canonical Wnt signaling pathway [GO:0090090]; positively regulated by positive regulation of canonical Wnt signaling pathway [GO:0090263] References: PMID:11532397, PMID:19619488 Definition: A type of Wnt signaling pathway in which Wnt binding to its receptor on the surface of a target cell results in the by propagation of the molecular signals via beta-catenin, and end with a change in transcription of target genes. In this pathway, the activated receptor signals via downstream effectors that result in the inhibition of beta-catenin phosphorylation, thereby preventing degradation of beta-catenin. Stabilized beta-catenin can then accumulate and travel to the nucleus to trigger changes in transcription of target genes. Relationships: is a type of Wnt signaling pathway [GO:0016055] Also known as: Wnt receptor signaling pathway through beta-catenin, Wnt receptor signaling pathway via beta-catenin, Wnt receptor signalling pathway through beta-catenin, canonical Wnt receptor signaling pathway, canonical Wnt-activated signaling pathway, frizzled-1 receptor signaling pathway Subtypes: canonical Wnt signaling pathway involved in negative regulation of apoptotic process [GO:0044336], canonical Wnt signaling pathway involved in positive regulation of apoptotic process [GO:0044337], canonical Wnt signaling pathway involved in mesenchymal stem cell differentiation [GO:0044338], canonical Wnt signaling pathway involved in heart development [GO:0061316]